{
  "gene": "UniProtKB:P26441",
  "term_label": "negative regulation of neuron apoptotic process",
  "gene_name": "Ciliary neurotrophic factor",
  "gene_symbol": "CNTF",
  "term_id": "GO:0043524"
}